{
  "gene_name": "Charged multivesicular body protein 4c",
  "gene": "UniProtKB:Q96CF2",
  "term_label": "nuclear membrane reassembly",
  "gene_symbol": "CHMP4C",
  "term_id": "GO:0031468"
}